{
  "gene_name": "Probable ubiquitin carboxyl-terminal hydrolase MINDY-4",
  "term_id": "UNKNOWN:0003",
  "term_label": "Unknown cellular component",
  "gene": "UniProtKB:Q4G0A6",
  "gene_symbol": "MINDY4"
}